{
  "term_id": "GO:0003725",
  "gene_name": "Double-stranded RNA-specific editase 1",
  "gene_symbol": "ADARB1",
  "term_label": "double-stranded RNA binding",
  "gene": "UniProtKB:P78563"
}